daunorubicin catabolic process [GO:1901770] (biological process) References: PMID:7601857 Sources: GOC:TermGenie, GOC:yaf Definition: The chemical reactions and pathways resulting in the breakdown of daunorubicin. Also known as: daunorubicin breakdown, daunorubicin catabolism, daunorubicin degradation Relationships: is a type of GO:0030640; is a type of aminoglycoside antibiotic catabolic process [GO:0030649]; is a type of ketone catabolic process [GO:0042182]; is a type of GO:0044597